{
  "gene_symbol": "RETSAT",
  "gene": "UniProtKB:Q6NUM9",
  "gene_name": "All-trans-retinol 13,14-reductase",
  "term_id": "GO:0051786",
  "term_label": "all-trans-retinol 13,14-reductase activity"
}